{
  "term_id": "GO:0005654",
  "term_label": "nucleoplasm",
  "gene_symbol": "RAD23A",
  "gene": "UniProtKB:P54725",
  "gene_name": "UV excision repair protein RAD23 homolog A"
}